{
  "gene_symbol": "TMEM127",
  "term_id": "GO:0016020",
  "gene_name": "Transmembrane protein 127",
  "term_label": "membrane",
  "gene": "UniProtKB:O75204"
}